{
  "gene_name": "Protein turtle homolog A",
  "gene": "UniProtKB:Q9P2J2",
  "term_label": "axon guidance",
  "gene_symbol": "IGSF9",
  "term_id": "GO:0007411"
}